{
  "term_label": "heart development",
  "term_id": "GO:0007507",
  "gene_symbol": "CFC1",
  "gene": "UniProtKB:P0CG37",
  "gene_name": "Cryptic protein"
}